membrane raft localization [GO:0051665] (biological process) Subtypes: membrane raft distribution [GO:0031580], plasma membrane raft localization [GO:0044856] Also known as: establishment and maintenance of membrane raft localization, lipid raft localization, membrane raft localisation References: PMID:16645198 Sources: GOC:ai Relationships: is a type of localization within membrane [GO:0051668] Definition: Any process in which membrane rafts are transported to, or maintained in, a specific location. Membrane rafts are small (10-200 nm), heterogeneous, highly dynamic, sterol- and sphingolipid-enriched membrane domains that compartmentalize cellular processes.